{
  "term_id": "GO:0000978",
  "term_label": "RNA polymerase II cis-regulatory region sequence-specific DNA binding",
  "gene": "UniProtKB:Q9UBP5",
  "gene_name": "Hairy_enhancer-of-split related with YRPW motif protein 2",
  "gene_symbol": "HEY2"
}